{
  "gene": "UniProtKB:Q9P0W0",
  "term_label": "type I interferon receptor binding",
  "term_id": "GO:0005132",
  "gene_name": "Interferon kappa",
  "gene_symbol": "IFNK"
}